{
  "gene": "UniProtKB:Q9UBG3",
  "gene_symbol": "CRNN",
  "term_id": "GO:0005509",
  "gene_name": "Cornulin",
  "term_label": "calcium ion binding"
}